{
  "gene": "UniProtKB:P45983",
  "term_label": "nucleus",
  "term_id": "GO:0005634",
  "gene_symbol": "MAPK8",
  "gene_name": "Mitogen-activated protein kinase 8"
}